{
  "gene_symbol": "SLC1A6",
  "gene_name": "Excitatory amino acid transporter 4",
  "term_label": "L-glutamate transmembrane transport",
  "term_id": "GO:0015813",
  "gene": "UniProtKB:P48664"
}